cardiac muscle cell fate determination [GO:0061442] (biological process) Definition: The process involved in cardiac muscle cell fate commitment. Once determination has taken place, a cell becomes committed to differentiate down a particular pathway regardless of its environment. Sources: GOC:BHF, GOC:dph Relationships: is a type of muscle cell fate determination [GO:0007521]; is a type of GO:0060913; is part of GO:0060923